{
  "term_label": "endocytosis",
  "gene_symbol": "REPS2",
  "gene": "UniProtKB:Q8NFH8",
  "term_id": "GO:0006897",
  "gene_name": "RalBP1-associated Eps domain-containing protein 2"
}